{
  "gene_symbol": "SCML1",
  "term_id": "GO:0005634",
  "gene": "UniProtKB:Q9UN30",
  "gene_name": "Sex comb on midleg-like protein 1",
  "term_label": "nucleus"
}